{
  "term_id": "GO:0000978",
  "gene": "UniProtKB:Q9NR83",
  "gene_name": "SLC2A4 regulator",
  "term_label": "RNA polymerase II cis-regulatory region sequence-specific DNA binding",
  "gene_symbol": "SLC2A4RG"
}